{
  "gene": "UniProtKB:Q96FM1",
  "gene_symbol": "PGAP3",
  "gene_name": "Post-GPI attachment to proteins factor 3",
  "term_label": "hydrolase activity, acting on ester bonds",
  "term_id": "GO:0016788"
}